{
  "term_label": "RNA polymerase II cis-regulatory region sequence-specific DNA binding",
  "term_id": "GO:0000978",
  "gene_name": "MHC class II regulatory factor RFX1",
  "gene": "UniProtKB:P22670",
  "gene_symbol": "RFX1"
}